paraxial mesoderm development [GO:0048339] (biological process) Definition: The process whose specific outcome is the progression of the paraxial mesoderm over time, from its formation to the mature structure. The paraxial mesoderm is the mesoderm located bilaterally adjacent to the notochord and neural tube. Sources: GOC:dgh Relationships: is a type of GO:0007498; is a type of mesenchyme development [GO:0060485]